{
  "gene_name": "Transmembrane protein 225",
  "term_label": "Unknown molecular function",
  "gene_symbol": "TMEM225",
  "term_id": "UNKNOWN:0001",
  "gene": "UniProtKB:Q6GV28"
}